{
  "term_label": "Unknown cellular component",
  "gene": "UniProtKB:O95497",
  "term_id": "UNKNOWN:0003",
  "gene_name": "Pantetheinase",
  "gene_symbol": "VNN1"
}